{
  "gene_name": "Disabled homolog 1",
  "term_label": "cytoplasm",
  "gene": "UniProtKB:O75553",
  "term_id": "GO:0005737",
  "gene_symbol": "DAB1"
}